{
  "term_label": "Cul3-RING ubiquitin ligase complex",
  "gene_name": "Kelch-like protein 11",
  "gene_symbol": "KLHL11",
  "gene": "UniProtKB:Q9NVR0",
  "term_id": "GO:0031463"
}